molting cycle, chitin-based cuticle [GO:0007591] (biological process) Also known as: chitin-based cuticle molting cycle Subtypes: GO:0007593 Relationships: is a type of molting cycle [GO:0042303] Definition: The periodic shedding of part or all of a chitin-based cuticle, which is then replaced by a new cuticle. An example of this is found in Drosophila melanogaster. Sources: GOC:jl, GOC:mtg_sensu